efflux pump complex [GO:1990281] (cellular component) Definition: A protein complex that is capable of efflux transmembrane transporter activity. References: PMID:21556065, PMID:9417051 Sources: GOC:dos Relationships: is a type of transmembrane transporter complex [GO:1902495] Also known as: efflux pump, efflux transmembrane transporter complex